{
  "term_label": "Unknown biological process",
  "gene": "UniProtKB:Q8N567",
  "gene_name": "Zinc finger CCHC domain-containing protein 9",
  "term_id": "UNKNOWN:0002",
  "gene_symbol": "ZCCHC9"
}